{
  "gene_symbol": "RRM2",
  "gene_name": "Ribonucleoside-diphosphate reductase subunit M2",
  "gene": "UniProtKB:P31350",
  "term_id": "GO:0005829",
  "term_label": "cytosol"
}